{
  "gene": "UniProtKB:Q7Z4T8",
  "term_label": "spermatid development",
  "gene_symbol": "GALNTL5",
  "term_id": "GO:0007286",
  "gene_name": "Inactive polypeptide N-acetylgalactosaminyltransferase-like protein 5"
}